regulation of parathyroid hormone secretion [GO:2000828] (biological process) Subtypes: GO:2000829, positive regulation of parathyroid hormone secretion [GO:2000830] Definition: Any process that modulates the frequency, rate or extent of parathyroid hormone secretion. Sources: GOC:obol Also known as: regulation of PTH secretion, regulation of parathormone secretion, regulation of parathyrin secretion Relationships: is a type of regulation of endocrine process [GO:0044060]; is a type of regulation of hormone secretion [GO:0046883]; regulates parathyroid hormone secretion [GO:0035898]